{
  "term_id": "UNKNOWN:0003",
  "term_label": "Unknown cellular component",
  "gene_symbol": "SGIP1",
  "gene": "UniProtKB:Q9BQI5",
  "gene_name": "SH3-containing GRB2-like protein 3-interacting protein 1"
}